{
  "gene": "UniProtKB:A0A0B4J200",
  "gene_name": "T cell receptor beta joining 2-3",
  "gene_symbol": "TRBJ2-3",
  "term_id": "UNKNOWN:0003",
  "term_label": "Unknown cellular component"
}